{
  "gene_symbol": "SRY",
  "gene": "UniProtKB:Q05066",
  "term_id": "GO:0001228",
  "gene_name": "Sex-determining region Y protein",
  "term_label": "DNA-binding transcription activator activity, RNA polymerase II-specific"
}